{
  "gene_symbol": "WASH4P",
  "gene_name": "Putative WAS protein family homolog 4",
  "term_label": "exocytosis",
  "term_id": "GO:0006887",
  "gene": "UniProtKB:A8MWX3"
}